{
  "gene": "UniProtKB:Q9BU20",
  "gene_symbol": "CPLANE2",
  "gene_name": "Ciliogenesis and planar polarity effector 2",
  "term_label": "GTPase activity",
  "term_id": "GO:0003924"
}